{
  "gene": "UniProtKB:Q8NET5",
  "gene_name": "NFAT activation molecule 1",
  "gene_symbol": "NFAM1",
  "term_label": "membrane raft",
  "term_id": "GO:0045121"
}